{
  "term_label": "osmosensory signaling pathway",
  "gene_name": "Transient receptor potential cation channel subfamily V member 3",
  "gene": "UniProtKB:Q8NET8",
  "gene_symbol": "TRPV3",
  "term_id": "GO:0007231"
}